{
  "gene_name": "DnaJ homolog subfamily A member 2",
  "gene_symbol": "DNAJA2",
  "term_label": "protein-folding chaperone binding",
  "term_id": "GO:0051087",
  "gene": "UniProtKB:O60884"
}